{
  "gene_symbol": "PTH2",
  "term_id": "UNKNOWN:0001",
  "gene": "UniProtKB:Q96A98",
  "term_label": "Unknown molecular function",
  "gene_name": "Tuberoinfundibular peptide of 39 residues"
}